{
  "gene": "UniProtKB:Q5T619",
  "gene_name": "Zinc finger protein 648",
  "term_label": "Unknown cellular component",
  "term_id": "UNKNOWN:0003",
  "gene_symbol": "ZNF648"
}